{
  "gene_symbol": "ZDHHC5",
  "gene": "UniProtKB:Q9C0B5",
  "term_label": "plasma membrane",
  "term_id": "GO:0005886",
  "gene_name": "Palmitoyltransferase ZDHHC5"
}